{
  "gene_symbol": "ZFAND4",
  "gene_name": "AN1-type zinc finger protein 4",
  "term_id": "UNKNOWN:0002",
  "gene": "UniProtKB:Q86XD8",
  "term_label": "Unknown biological process"
}